negative regulation of respiratory burst involved in inflammatory response [GO:0060266] (biological process) Sources: GOC:BHF, GOC:dph, GOC:tb Also known as: negative regulation of respiratory burst involved in acute inflammatory response Definition: Any process that decreases the rate, frequency or extent of a phase of elevated metabolic activity, during which oxygen consumption increases made as a defense response ; this leads to the production, by an NADH dependent system, of hydrogen peroxide (H2O2), superoxide anions and hydroxyl radicals. Relationships: is a type of negative regulation of immune effector process [GO:0002698]; is a type of negative regulation of innate immune response [GO:0045824]; is a type of GO:0050728; is a type of negative regulation of multicellular organismal process [GO:0051241]; is a type of GO:0060264; is a type of GO:0060268; is a type of regulation of cell development [GO:0060284]; negatively regulates respiratory burst involved in inflammatory response [GO:0002536]